guanine salvage [GO:0006178] (biological process) Definition: Any process that generates guanine, 2-amino-6-hydroxypurine, from derivatives of it without de novo synthesis. Also known as: guanine, xanthine and their nucleoside salvage Sources: GOC:jl Relationships: is a type of purine nucleobase salvage [GO:0043096]; is a type of guanine biosynthetic process [GO:0046099]